insulin-responsive compartment [GO:0032593] (cellular component) Also known as: GLUT4 storage compartment, GSC, IRC References: PMID:17644329 Definition: A small membrane-bounded vesicle that releases its contents by exocytosis in response to insulin stimulation; the contents are enriched in GLUT4, IRAP and VAMP2. Relationships: is a type of secretory granule [GO:0030141]